isocitrate lyase activity [GO:0004451] (molecular function) Also known as: ICL activity, isocitrase activity, isocitratase activity, isocitrate glyoxylate-lyase (succinate-forming), isocitrate glyoxylate-lyase activity, isocitritase activity, threo-DS-isocitrate glyoxylate-lyase activity Definition: Catalysis of the reaction: isocitrate = glyoxylate + succinate. Sources: EC:4.1.3.1, RHEA:13245 Relationships: is a type of oxo-acid-lyase activity [GO:0016833]